{
  "term_id": "UNKNOWN:0001",
  "term_label": "Unknown molecular function",
  "gene_name": "Ubiquitin-associated domain-containing protein 1",
  "gene": "UniProtKB:Q9BSL1",
  "gene_symbol": "UBAC1"
}